negative regulation of leaf senescence [GO:1900056] (biological process) Sources: GOC:TermGenie Relationships: is a type of GO:0051093; is a type of regulation of leaf senescence [GO:1900055]; negatively regulates leaf senescence [GO:0010150] Definition: Any process that stops, prevents or reduces the frequency, rate or extent of leaf senescence. Also known as: down regulation of leaf senescence, down-regulation of leaf senescence, downregulation of leaf senescence, inhibition of leaf senescence